genomic imprinting [GO:0071514] (biological process) Definition: The establishment of epigenetic modifications (imprints) during gametogenesis, and propagation of these imprints during the organism's life. Genomic imprinting leads to an asymmetry between the maternal and paternal alleles and differential expression of the corresponding alleles. This can happen through heterochromatin formation or differential chromatin loop formation. References: PMID:24492710, PMID:31896690, PMID:31965998 Relationships: is_a epigenetic programming of gene expression [GO:0043045]; is part of germ cell development [GO:0007281] Subtypes: GO:0060818, epigenetic programming in the central cell [GO:0141063], autosome genomic imprinting [GO:0141068] Also known as: DNA imprinting, establishment of genomic imprinting, genetic imprinting